{
  "gene_symbol": "COQ6",
  "gene_name": "Ubiquinone biosynthesis monooxygenase COQ6, mitochondrial",
  "term_label": "ubiquinone biosynthetic process",
  "term_id": "GO:0006744",
  "gene": "UniProtKB:Q9Y2Z9"
}